RNA 2'-O-ribose methylation guide activity [GO:0030561] (molecular function) Definition: Specifies the site of 2'-O-ribose methylation in an RNA molecule by base pairing with a short sequence around the target residue. Relationships: is a type of RNA modification guide activity [GO:0030555] Note: Note that this term describes the activity of a nucleic acid, usually RNA, gene product that interacts with other RNA molecules via base pairing; it should not be used to annotate proteins. Subtypes: rRNA 2'-O-ribose methylation guide activity [GO:0030562], snRNA 2'-O-ribose methylation guide activity [GO:0030563], tRNA 2'-O-ribose methylation guide activity [GO:0030564] References: PMID:12457565 Sources: GOC:mah